{
  "gene_symbol": "PDE3A",
  "term_label": "negative regulation of cAMP/PKA signal transduction",
  "gene_name": "cGMP-inhibited 3',5'-cyclic phosphodiesterase 3A",
  "term_id": "GO:0141162",
  "gene": "UniProtKB:Q14432"
}